{
  "term_id": "GO:0003924",
  "term_label": "GTPase activity",
  "gene_symbol": "RHOT1",
  "gene": "UniProtKB:Q8IXI2",
  "gene_name": "Mitochondrial Rho GTPase 1"
}